{
  "term_label": "neuron fate specification",
  "term_id": "GO:0048665",
  "gene_symbol": "ISL2",
  "gene": "UniProtKB:Q96A47",
  "gene_name": "Insulin gene enhancer protein ISL-2"
}